{
  "gene_symbol": "CRYBG2",
  "gene_name": "Beta_gamma crystallin domain-containing protein 2",
  "term_id": "UNKNOWN:0003",
  "term_label": "Unknown cellular component",
  "gene": "UniProtKB:Q8N1P7"
}